{
  "gene_name": "Single-pass membrane and coiled-coil domain-containing protein 2",
  "term_id": "UNKNOWN:0001",
  "gene_symbol": "SMCO2",
  "term_label": "Unknown molecular function",
  "gene": "UniProtKB:A6NFE2"
}